{
  "term_label": "cytoplasm",
  "gene_name": "Ubiquitin carboxyl-terminal hydrolase 44",
  "term_id": "GO:0005737",
  "gene": "UniProtKB:Q9H0E7",
  "gene_symbol": "USP44"
}